entry into host through the stromata [GO:0140717] (biological process) Relationships: is a type of GO:0044409 References: PMID:16959560, PMID:17419713, PMID:29307013 Definition: Entry of a symbiont into host plant tissue via the stromata, microscopic pores in the epidermis of the aerial parts of terrestrial plants. These pores are essential for photosynthesis, as they allow CO2 to diffuse into the plant. The host is defined as the larger of the organisms involved in a symbiotic interaction.